{
  "gene_symbol": "GABRE",
  "gene_name": "Gamma-aminobutyric acid receptor subunit epsilon",
  "term_id": "GO:0022851",
  "term_label": "GABA-gated chloride ion channel activity",
  "gene": "UniProtKB:P78334"
}